{
  "term_label": "Unknown cellular component",
  "gene_symbol": "TRAJ46",
  "gene_name": "T cell receptor alpha joining 46 (Fragment)",
  "term_id": "UNKNOWN:0003",
  "gene": "UniProtKB:A0A075B6W4"
}